{
  "gene_name": "Hepatitis A virus cellular receptor 1",
  "term_id": "GO:0033005",
  "gene_symbol": "HAVCR1",
  "term_label": "positive regulation of mast cell activation",
  "gene": "UniProtKB:Q96D42"
}